{
  "gene_name": "Coiled-coil domain-containing protein 102A",
  "term_id": "UNKNOWN:0002",
  "gene": "UniProtKB:Q96A19",
  "term_label": "Unknown biological process",
  "gene_symbol": "CCDC102A"
}